protein-arginine omega-N monomethyltransferase activity [GO:0035241] (MF) Definition: Catalysis of the addition of a methyl group to either of the unmethylated terminal nitrogen atoms (also called omega nitrogen) in peptidyl-arginine to form an omega-N-G-monomethylated arginine residue. The reaction is S-adenosyl-L-methionine + [protein]-L-arginine = S-adenosyl-L-homocysteine + [protein]-Nomega-methyl-L-arginine. References: PMID:14705965 Sources: EC:2.1.1.321, RESID:AA0069 Also known as: protein arginine omega-N monomethylase activity, S-adenosyl-L-methionine:[protein]-L-arginine N-methyltransferase ([protein]-Nomega-methyl-L-arginine-forming), type III protein arginine methyltransferase activity Note: Type III protein arginine methyltransferases catalyze the single methylation of one of the terminal nitrogen atoms of the guanidino group in an L-arginine residue within a protein. Unlike type I and type II protein arginine methyltransferases, which also catalyze this reaction, type III enzymes do not methylate the substrate any further. Relationships: is a type of protein-arginine N-methyltransferase activity [GO:0016274]